{
  "gene_symbol": "LRP2BP",
  "gene_name": "LRP2-binding protein",
  "gene": "UniProtKB:Q9P2M1",
  "term_id": "UNKNOWN:0003",
  "term_label": "Unknown cellular component"
}